{
  "gene_name": "Programmed cell death 6-interacting protein",
  "term_label": "Unknown molecular function",
  "gene_symbol": "PDCD6IP",
  "term_id": "UNKNOWN:0001",
  "gene": "UniProtKB:Q8WUM4"
}